{
  "term_label": "reticulophagy",
  "gene": "UniProtKB:Q86WV6",
  "term_id": "GO:0061709",
  "gene_name": "Stimulator of interferon genes protein",
  "gene_symbol": "STING1"
}